wound healing, spreading of cells [GO:0044319] (biological process) Sources: GOC:jl Relationships: is a type of GO:0016477; BFO_0000050 epiboly involved in wound healing [GO:0090505] Subtypes: GO:0035313 Also known as: cell migration involved in wound healing epiboly Definition: The migration of a cell along or through a wound gap that contributes to the reestablishment of a continuous surface.